{
  "gene_name": "Transmembrane emp24 domain-containing protein 9",
  "term_label": "COPII-coated ER to Golgi transport vesicle",
  "gene": "UniProtKB:Q9BVK6",
  "term_id": "GO:0030134",
  "gene_symbol": "TMED9"
}